{
  "term_id": "GO:2000738",
  "gene_symbol": "TACSTD2",
  "gene_name": "Tumor-associated calcium signal transducer 2",
  "gene": "UniProtKB:P09758",
  "term_label": "positive regulation of stem cell differentiation"
}